{
  "term_label": "Unknown cellular component",
  "gene": "UniProtKB:P17040",
  "gene_symbol": "ZSCAN20",
  "gene_name": "Zinc finger and SCAN domain-containing protein 20",
  "term_id": "UNKNOWN:0003"
}